positive regulation of muscle organ development [GO:0048636] (BP) Sources: GOC:go_curators Relationships: is a type of regulation of muscle organ development [GO:0048634]; is a type of GO:0051094; is_a positive regulation of multicellular organismal process [GO:0051240]; positively regulates muscle organ development [GO:0007517] Subtypes: positive regulation of somitomeric trunk muscle development [GO:0014709], GO:0045844 Definition: Any process that activates, maintains or increases the rate of muscle development. Also known as: up regulation of muscle development, up-regulation of muscle development, upregulation of muscle development, activation of muscle development, stimulation of muscle development